{
  "term_id": "GO:0005615",
  "gene": "UniProtKB:P17405",
  "gene_symbol": "SMPD1",
  "gene_name": "Sphingomyelin phosphodiesterase",
  "term_label": "extracellular space"
}